{
  "gene_symbol": "ASCC1",
  "term_label": "Unknown molecular function",
  "gene_name": "Activating signal cointegrator 1 complex subunit 1",
  "gene": "UniProtKB:Q8N9N2",
  "term_id": "UNKNOWN:0001"
}